{
  "gene_name": "Golgin subfamily A member 6D",
  "gene_symbol": "GOLGA6D",
  "gene": "UniProtKB:P0CG33",
  "term_id": "UNKNOWN:0001",
  "term_label": "Unknown molecular function"
}